{
  "gene_symbol": "OR13C4",
  "gene_name": "Olfactory receptor 13C4",
  "term_id": "GO:0050911",
  "gene": "UniProtKB:Q8NGS5",
  "term_label": "detection of chemical stimulus involved in sensory perception of smell"
}